shikimate transmembrane transporter activity [GO:0015530] (molecular function) Sources: GOC:ai Relationships: is a type of monocarboxylic acid transmembrane transporter activity [GO:0008028]; is part of shikimate transmembrane transport [GO:0015733] Subtypes: shikimate:proton symporter activity [GO:0015533] Definition: Enables the transfer of shikimate from one side of a membrane to the other. Shikimate is an important intermediate in the biosynthesis of aromatic amino acids.